{
  "term_id": "UNKNOWN:0001",
  "term_label": "Unknown molecular function",
  "gene_name": "BTB_POZ domain-containing protein 19",
  "gene_symbol": "BTBD19",
  "gene": "UniProtKB:C9JJ37"
}